{
  "gene_symbol": "SERPINE1",
  "gene": "UniProtKB:P05121",
  "gene_name": "Plasminogen activator inhibitor 1",
  "term_label": "serine-type endopeptidase inhibitor activity",
  "term_id": "GO:0004867"
}